{
  "term_id": "GO:0005634",
  "gene": "UniProtKB:P11308",
  "gene_symbol": "ERG",
  "gene_name": "Transcriptional regulator ERG",
  "term_label": "nucleus"
}